{
  "term_id": "GO:0043023",
  "gene_symbol": "LTN1",
  "gene": "UniProtKB:O94822",
  "term_label": "ribosomal large subunit binding",
  "gene_name": "E3 ubiquitin-protein ligase listerin"
}